{
  "gene_symbol": "MRPL12",
  "term_label": "structural constituent of ribosome",
  "gene": "UniProtKB:P52815",
  "term_id": "GO:0003735",
  "gene_name": "Large ribosomal subunit protein bL12m"
}